regulation of interleukin-34 production [GO:0150157] (biological process) Definition: Any process that modulates the frequency, rate or extent of interleukin-34 production. Also known as: interleukin-34 biosynthetic process, regulation of interleukin-34 biosynthetic process Relationships: is a type of regulation of cytokine production [GO:0001817]; regulates interleukin-34 production [GO:0150155] Subtypes: GO:0150158, GO:0150159 References: PMID:26754294 Sources: GOC:aruk